DNA replication proofreading [GO:0045004] (biological process) Relationships: is a type of DNA repair [GO:0006281]; is a type of DNA-templated DNA replication maintenance of fidelity [GO:0045005] Definition: Correction of replication errors by DNA polymerase using a 3'-5' exonuclease activity. Sources: GOC:ai